{
  "term_label": "phosphatidylinositol-3-phosphate phosphatase activity",
  "gene_symbol": "MTMR3",
  "term_id": "GO:0004438",
  "gene": "UniProtKB:Q13615",
  "gene_name": "Myotubularin-related protein 3"
}